{
  "gene_name": "Serine_arginine repetitive matrix protein 4",
  "term_label": "mRNA binding",
  "gene_symbol": "SRRM4",
  "gene": "UniProtKB:A7MD48",
  "term_id": "GO:0003729"
}